{
  "gene_name": "Multifunctional methyltransferase subunit TRM112-like protein",
  "term_label": "maturation of LSU-rRNA",
  "gene_symbol": "TRMT112",
  "gene": "UniProtKB:Q9UI30",
  "term_id": "GO:0000470"
}